{
  "gene": "UniProtKB:Q96EX1",
  "term_id": "UNKNOWN:0003",
  "gene_symbol": "SMIM12",
  "gene_name": "Small integral membrane protein 12",
  "term_label": "Unknown cellular component"
}